{
  "gene_name": "Proline and serine-rich protein 3",
  "term_id": "UNKNOWN:0003",
  "term_label": "Unknown cellular component",
  "gene_symbol": "PROSER3",
  "gene": "UniProtKB:Q2NL68"
}